embryonic heart tube left/right pattern formation [GO:0060971] (biological process) Sources: GOC:mtg_heart Definition: The pattern specification process that results in the subdivision of the left/right axis of the embryonic heart tube in space to define an area or volume in which specific patterns of cell differentiation will take place. Relationships: is a type of left/right pattern formation [GO:0060972]; is part of embryonic heart tube development [GO:0035050]